activation of NF-kappaB-inducing kinase activity [GO:0007250] (biological process) Definition: The stimulation of the activity of NF-kappaB-inducing kinase through phosphorylation at specific residues. References: PMID:12773372 Sources: GOC:jl Also known as: positive regulation of NF-kappaB-inducing kinase activity, activation of NIK activity Relationships: is a type of GO:0032147; is part of non-canonical NF-kappaB signal transduction [GO:0038061]